{
  "gene_name": "Putative cytochrome P450 family member 4F30",
  "term_label": "Unknown biological process",
  "term_id": "UNKNOWN:0002",
  "gene": "UniProtKB:Q9H0H9",
  "gene_symbol": "CYP4F30P"
}